{
  "gene": "UniProtKB:P62487",
  "gene_name": "DNA-directed RNA polymerase II subunit RPB7",
  "term_label": "RNA polymerase II, core complex",
  "gene_symbol": "POLR2G",
  "term_id": "GO:0005665"
}